{
  "gene": "UniProtKB:P26373",
  "term_label": "structural constituent of ribosome",
  "term_id": "GO:0003735",
  "gene_symbol": "RPL13",
  "gene_name": "Large ribosomal subunit protein eL13"
}